{
  "term_label": "mediator complex",
  "gene_symbol": "MED11",
  "gene": "UniProtKB:Q9P086",
  "term_id": "GO:0016592",
  "gene_name": "Mediator of RNA polymerase II transcription subunit 11"
}